{
  "gene_name": "Aggrecan core protein",
  "term_label": "Unknown molecular function",
  "gene": "UniProtKB:P16112",
  "gene_symbol": "ACAN",
  "term_id": "UNKNOWN:0001"
}